{
  "gene": "UniProtKB:E9PRG8",
  "term_id": "UNKNOWN:0003",
  "gene_name": "Uncharacterized protein C11orf98",
  "term_label": "Unknown cellular component",
  "gene_symbol": "C11orf98"
}